{
  "term_id": "UNKNOWN:0003",
  "gene_name": "Olfactory receptor 8B12",
  "gene": "UniProtKB:Q8NGG6",
  "term_label": "Unknown cellular component",
  "gene_symbol": "OR8B12"
}